host-mediated activation of viral RNA-templated transcription [GO:0140181] (biological process) Definition: A process in which a host organism initiates, promotes, or enhances the normal execution of viral RNA-templated transcription, the synthesis of either RNA on a RNA template. Relationships: is a type of host-mediated activation of viral transcription [GO:0043923] References: PMID:18836083 Also known as: positive regulation by host of viral RNA-templated transcription, positive regulation of viral RNA-templated transcription by host